{
  "gene_name": "Protein FAM91A1",
  "term_id": "UNKNOWN:0001",
  "gene": "UniProtKB:Q658Y4",
  "gene_symbol": "FAM91A1",
  "term_label": "Unknown molecular function"
}